{
  "term_id": "UNKNOWN:0002",
  "gene_symbol": "GAGE1",
  "gene_name": "G antigen 1",
  "gene": "UniProtKB:P0DTW1",
  "term_label": "Unknown biological process"
}